{
  "term_label": "intracellular signal transduction",
  "gene_symbol": "MAST2",
  "gene_name": "Microtubule-associated serine_threonine-protein kinase 2",
  "gene": "UniProtKB:Q6P0Q8",
  "term_id": "GO:0035556"
}